{
  "term_id": "GO:0098609",
  "gene_name": "Contactin-5",
  "term_label": "cell-cell adhesion",
  "gene": "UniProtKB:O94779",
  "gene_symbol": "CNTN5"
}